{
  "term_id": "GO:0005802",
  "gene": "UniProtKB:O75379",
  "gene_name": "Vesicle-associated membrane protein 4",
  "term_label": "trans-Golgi network",
  "gene_symbol": "VAMP4"
}